{
  "term_label": "Unknown molecular function",
  "gene": "UniProtKB:Q92932",
  "term_id": "UNKNOWN:0001",
  "gene_symbol": "PTPRN2",
  "gene_name": "Receptor-type tyrosine-protein phosphatase N2"
}